{
  "term_label": "HULC complex",
  "gene_symbol": "UBE2U",
  "term_id": "GO:0033503",
  "gene_name": "Ubiquitin-conjugating enzyme E2 U",
  "gene": "UniProtKB:Q5VVX9"
}